{
  "term_id": "GO:0016192",
  "term_label": "vesicle-mediated transport",
  "gene": "UniProtKB:Q8N9I0",
  "gene_name": "Synaptotagmin-2",
  "gene_symbol": "SYT2"
}